terrequinone A biosynthetic process [GO:1900796] (biological process) Also known as: terrequinone A metabolic process, terrequinone A metabolism, terrequinone A anabolism, terrequinone A biosynthesis, terrequinone A formation, terrequinone A synthesis References: PMID:17291795, PMID:17704773 Sources: GOC:TermGenie, GOC:di Regulation: positively regulated by GO:1900854 Definition: The chemical reactions and pathways resulting in the formation of terrequinone A. Relationships: is a type of alkaloid biosynthetic process [GO:0009821]; is a type of olefinic compound biosynthetic process [GO:0120255]; is a type of quinone biosynthetic process [GO:1901663]